{
  "gene": "UniProtKB:Q9NR55",
  "term_label": "DNA-binding transcription factor activity, RNA polymerase II-specific",
  "term_id": "GO:0000981",
  "gene_symbol": "BATF3",
  "gene_name": "Basic leucine zipper transcriptional factor ATF-like 3"
}